uridine transmembrane transporter activity [GO:0015213] (MF) Relationships: is a type of pyrimidine nucleoside transmembrane transporter activity [GO:0015214]; is part of GO:0015862 Definition: Enables the transfer of uridine, uracil riboside, from one side of a membrane to the other. Sources: GOC:go_curators Subtypes: GO:0015394 Also known as: uracil/uridine permease activity